{
  "gene": "UniProtKB:P16471",
  "term_id": "GO:0009897",
  "gene_name": "Prolactin receptor",
  "gene_symbol": "PRLR",
  "term_label": "external side of plasma membrane"
}